{
  "gene_symbol": "AGO4",
  "term_label": "cytoplasmic ribonucleoprotein granule",
  "gene": "UniProtKB:Q9HCK5",
  "term_id": "GO:0036464",
  "gene_name": "Protein argonaute-4"
}